{
  "term_label": "actin binding",
  "gene": "UniProtKB:Q765P7",
  "gene_name": "Protein MTSS 2",
  "gene_symbol": "MTSS2",
  "term_id": "GO:0003779"
}